{
  "gene_symbol": "ZNF331",
  "gene": "UniProtKB:Q9NQX6",
  "term_id": "GO:0000981",
  "term_label": "DNA-binding transcription factor activity, RNA polymerase II-specific",
  "gene_name": "Zinc finger protein 331"
}